positive regulation of ergot alkaloid biosynthetic process [GO:1900824] (BP) Sources: GOC:TermGenie, GOC:di Subtypes: positive regulation of chanoclavine-I aldehyde biosynthetic process [GO:1900648], positive regulation of fumigaclavine C biosynthetic process [GO:1900839] Also known as: activation of ergot alkaloid anabolism, activation of ergot alkaloid biosynthesis, activation of ergot alkaloid formation, activation of ergot alkaloid synthesis, positive regulation of ergot alkaloid anabolism, positive regulation of ergot alkaloid biosynthesis, positive regulation of ergot alkaloid formation, positive regulation of ergot alkaloid synthesis, up regulation of ergot alkaloid anabolism, up regulation of ergot alkaloid biosynthesis, up regulation of ergot alkaloid biosynthetic process, up regulation of ergot alkaloid formation, up regulation of ergot alkaloid synthesis, up-regulation of ergot alkaloid anabolism, up-regulation of ergot alkaloid biosynthesis, up-regulation of ergot alkaloid biosynthetic process, up-regulation of ergot alkaloid formation, up-regulation of ergot alkaloid synthesis, upregulation of ergot alkaloid anabolism, upregulation of ergot alkaloid biosynthesis, upregulation of ergot alkaloid biosynthetic process, upregulation of ergot alkaloid formation, upregulation of ergot alkaloid synthesis, activation of ergot alkaloid biosynthetic process Relationships: is a type of positive regulation of secondary metabolite biosynthetic process [GO:1900378]; is a type of regulation of ergot alkaloid biosynthetic process [GO:1900822]; positively regulates ergot alkaloid biosynthetic process [GO:0035837] Definition: Any process that activates or increases the frequency, rate or extent of ergot alkaloid biosynthetic process.